{
  "gene": "UniProtKB:P56704",
  "gene_name": "Protein Wnt-3a",
  "term_id": "GO:0060070",
  "gene_symbol": "WNT3A",
  "term_label": "canonical Wnt signaling pathway"
}